{
  "term_id": "GO:0005737",
  "gene_name": "Arrestin domain-containing protein 1",
  "term_label": "cytoplasm",
  "gene_symbol": "ARRDC1",
  "gene": "UniProtKB:Q8N5I2"
}